{
  "term_id": "GO:0043524",
  "gene_name": "Neurotrophin-4",
  "term_label": "negative regulation of neuron apoptotic process",
  "gene": "UniProtKB:P34130",
  "gene_symbol": "NTF4"
}